{
  "gene_name": "5'-AMP-activated protein kinase subunit gamma-3",
  "gene_symbol": "PRKAG3",
  "term_id": "GO:0019887",
  "gene": "UniProtKB:Q9UGI9",
  "term_label": "protein kinase regulator activity"
}